positive regulation of macrophage inflammatory protein-1 gamma production [GO:0071648] (biological process) Also known as: positive regulation of CCL9 production, positive regulation of MIP-1g production, positive regulation of chemokine (C-C motif) ligand 9 production Sources: GOC:mah Relationships: is a type of GO:0032722; is a type of GO:0071646; positively regulates macrophage inflammatory protein-1 gamma production [GO:0071607] Definition: Any process that activates or increases the frequency, rate, or extent of production of macrophage inflammatory protein-1 gamma.